lipoxin B4 biosynthetic process [GO:2001306] (biological process) Definition: The chemical reactions and pathways resulting in the formation of lipoxin B4. Lipoxin B4 is a C20 hydroxy fatty acid having (5S)-, (14R)- and (15S)-hydroxy groups as well as (6E)- (8Z)-, (10E)- and (12E)-double bonds. Sources: GOC:mw Also known as: LXB4 anabolism, LXB4 biosynthesis, LXB4 biosynthetic process, LXB4 formation, LXB4 synthesis, lipoxin B4 anabolism, lipoxin B4 biosynthesis, lipoxin B4 formation, lipoxin B4 synthesis Relationships: is a type of GO:0006636; is a type of long-chain fatty acid biosynthetic process [GO:0042759]; is a type of lipoxin biosynthetic process [GO:2001301]; is a type of lipoxin B4 metabolic process [GO:2001304]